{
  "gene": "UniProtKB:A8MTL0",
  "gene_symbol": "IQCF5",
  "term_id": "UNKNOWN:0003",
  "term_label": "Unknown cellular component",
  "gene_name": "IQ domain-containing protein F5"
}